{
  "gene_symbol": "BRINP1",
  "gene": "UniProtKB:O60477",
  "gene_name": "BMP_retinoic acid-inducible neural-specific protein 1",
  "term_label": "Unknown molecular function",
  "term_id": "UNKNOWN:0001"
}